mesendoderm migration [GO:0090133] (biological process) Sources: GOC:ascb_2009, GOC:dph, GOC:tb Relationships: is a type of epithelium migration [GO:0090132]; is part of GO:0007369; is part of GO:0048382 Definition: The process in which the population of cells that make up a mesendoderm undergo directed movement. The mesendoderm is the epithelial tissue that gives rise to both mesoderm and endoderm.